TERT-RMRP complex [GO:1990572] (cellular component) Relationships: is a type of GO:0031379; is a type of ribonucleoprotein complex [GO:1990904] Definition: A ribonucleoprotein complex that has RNA-directed RNA polymerase (RdRP) activity, and is composed of telomerase reverse transcriptase (TERT) and the non-coding RNA component of mitochondrial RNA processing endoribonuclease (RMRP). References: PMID:19701182 Sources: GOC:BHF, GOC:BHF_telomere, GOC:bf, GOC:nc Also known as: telomerase reverse transcriptase:RMRP RNA complex